{
  "term_label": "Unknown cellular component",
  "gene_name": "Putative TBC1 domain family member 29",
  "gene": "UniProtKB:Q9UFV1",
  "gene_symbol": "TBC1D29P",
  "term_id": "UNKNOWN:0003"
}